response to cyclosporin A [GO:1905237] (biological process) Definition: Any process that results in a change in state or activity of a cell or an organism (in terms of movement, secretion, enzyme production, gene expression, etc.) as a result of a cyclosporin A stimulus. References: PMID:24914722 Sources: GOC:TermGenie, GO_REF:0000071 Relationships: is a type of GO:1901698; is a type of response to oxygen-containing compound [GO:1901700] Subtypes: cellular response to cyclosporin A [GO:1905238] Also known as: response to cyclophilin